{
  "term_label": "glycerol metabolic process",
  "term_id": "GO:0006071",
  "gene_symbol": "GK5",
  "gene_name": "Putative glycerol kinase 5",
  "gene": "UniProtKB:Q6ZS86"
}